{
  "gene_name": "Chemerin-like receptor 2",
  "term_id": "GO:0043005",
  "gene": "UniProtKB:P46091",
  "gene_symbol": "CMKLR2",
  "term_label": "neuron projection"
}